{
  "gene_symbol": "SMIM39",
  "gene": "UniProtKB:A0A1B0GW54",
  "gene_name": "Small integral membrane protein 39",
  "term_label": "Unknown cellular component",
  "term_id": "UNKNOWN:0003"
}